negative regulation of cytokine production involved in inflammatory response [GO:1900016] (biological process) Definition: Any process that stops, prevents or reduces the frequency, rate or extent of cytokine production involved in inflammatory response. Also known as: down regulation of cytokine production involved in acute inflammatory response, negative regulation of cytokine production involved in acute inflammatory response, down regulation of cytokine production involved in inflammatory response Sources: GOC:TermGenie Relationships: is a type of negative regulation of cytokine production [GO:0001818]; is a type of regulation of cytokine production involved in inflammatory response [GO:1900015]; negatively regulates GO:0002534